{
  "term_label": "acetylcholine-gated channel complex",
  "gene": "UniProtKB:P30532",
  "gene_symbol": "CHRNA5",
  "term_id": "GO:0005892",
  "gene_name": "Neuronal acetylcholine receptor subunit alpha-5"
}